mitochondrion-mitochondrion outer membrane tether activity [GO:0160204] (MF) Definition: The binding activity of a molecule that brings together two mitochondrion membranes via membrane lipid binding or by interacting with a mitochondrial outer membrane protein, to establish or maintain the localization of the mitochondrion. Relationships: is a type of protein-membrane adaptor activity [GO:0043495] Also known as: mitochondrion membrane tether activity, mitochondrion outer membrane tether activity References: PMID:38843396